{
  "gene": "UniProtKB:Q8IYD8",
  "term_label": "double-strand break repair via synthesis-dependent strand annealing",
  "gene_symbol": "FANCM",
  "term_id": "GO:0045003",
  "gene_name": "Fanconi anemia group M protein"
}